{
  "gene_name": "Stonin-2",
  "term_label": "cytosol",
  "gene": "UniProtKB:Q8WXE9",
  "gene_symbol": "STON2",
  "term_id": "GO:0005829"
}